{
  "gene": "UniProtKB:O95754",
  "gene_name": "Semaphorin-4F",
  "term_label": "axon guidance",
  "term_id": "GO:0007411",
  "gene_symbol": "SEMA4F"
}